{
  "gene_symbol": "SLC27A4",
  "term_id": "GO:0044539",
  "term_label": "long-chain fatty acid import into cell",
  "gene_name": "Long-chain fatty acid transport protein 4",
  "gene": "UniProtKB:Q6P1M0"
}